{
  "term_id": "GO:0000978",
  "term_label": "RNA polymerase II cis-regulatory region sequence-specific DNA binding",
  "gene_symbol": "PAX2",
  "gene": "UniProtKB:Q02962",
  "gene_name": "Paired box protein Pax-2"
}